{
  "gene_name": "Beta-actin-like protein 2",
  "term_id": "GO:0019901",
  "term_label": "protein kinase binding",
  "gene": "UniProtKB:Q562R1",
  "gene_symbol": "ACTBL2"
}